{
  "gene_name": "Transitional endoplasmic reticulum ATPase",
  "term_label": "polyubiquitin modification-dependent protein binding",
  "gene": "UniProtKB:P55072",
  "gene_symbol": "VCP",
  "term_id": "GO:0031593"
}